{
  "gene": "UniProtKB:P0C860",
  "gene_name": "Putative male-specific lethal-3 protein-like 2",
  "term_label": "MSL complex",
  "gene_symbol": "MSL3B",
  "term_id": "GO:0072487"
}